{
  "term_id": "GO:0006626",
  "gene_name": "Mitochondrial fission factor",
  "gene": "UniProtKB:Q9GZY8",
  "gene_symbol": "MFF",
  "term_label": "protein targeting to mitochondrion"
}